{
  "gene_name": "Aldo-keto reductase family 1 member C1",
  "term_label": "aldose reductase (NADPH) activity",
  "term_id": "GO:0004032",
  "gene_symbol": "AKR1C1",
  "gene": "UniProtKB:Q04828"
}